S-lactaldehyde reductase activity [GO:0052661] (molecular function) Sources: RHEA:15933 Also known as: (S)-propane-1,2-diol:NAD+ oxidoreductase activity, L-lactaldehyde:propanediol oxidoreductase activity Relationships: is a type of GO:0008912 Definition: Catalysis of the reaction: (S)-propane-1,2-diol + NAD+ = (S)-lactaldehyde + NADH + H+.